cytoplasmic side of mitochondrial outer membrane [GO:0032473] (cellular component) Also known as: cytosolic side of mitochondrial outer membrane, external leaflet of mitochondrial outer membrane, external side of mitochondrial outer membrane, external side of mitochondrial envelope Sources: GOC:mah Note: In GO, 'external side' still refers to part of the membrane and does not refer to components beyond (outside of) the membrane. Relationships: is_a cytoplasmic side of membrane [GO:0098562]; is part of GO:0005741 Definition: The external (cytoplasmic) face of the mitochondrial outer membrane.